{
  "gene_symbol": "CCL2",
  "term_id": "GO:0048020",
  "term_label": "CCR chemokine receptor binding",
  "gene_name": "C-C motif chemokine 2",
  "gene": "UniProtKB:P13500"
}